cell-cell signaling involved in lung development [GO:0060495] (biological process) Subtypes: GO:0060496, epithelial-mesenchymal cell signaling involved in lung development [GO:0061111], mesothelial-mesenchymal cell signaling involved in early lung development [GO:0061142] Definition: Any process that mediates the transfer of information from one cell to another and contributes to the progression of the lung, from its initial state to the mature structure. Sources: GOC:dph, GOC:mtg_lung Also known as: cell-cell signalling involved in lung development Relationships: is a type of GO:0007267; is part of GO:0030324